{
  "gene": "UniProtKB:P0DMV0",
  "term_label": "Unknown biological process",
  "gene_symbol": "CT45A7",
  "term_id": "UNKNOWN:0002",
  "gene_name": "Cancer_testis antigen family 45 member A7"
}